glycosylphosphatidylinositol-mannosyltransferase II complex [GO:0120097] (CC) Also known as: GPI-MT-I complex Relationships: is a type of mannosyltransferase complex [GO:0031501]; is a type of endoplasmic reticulum protein-containing complex [GO:0140534] References: PMID:17615295 Sources: GOC:bhm Definition: A protein complex that is involved in the transfer of the second mannose to the glycosylphosphatidylinositol (GPI) during GPI precursor assembly. In yeast S. cerevisiae this complex consists of GPI18p and PGA1p.